{
  "term_id": "GO:0005739",
  "gene_name": "Armadillo repeat-containing protein 10",
  "gene": "UniProtKB:Q8N2F6",
  "gene_symbol": "ARMC10",
  "term_label": "mitochondrion"
}